{
  "gene_symbol": "RASEF",
  "term_label": "vesicle-mediated transport",
  "gene": "UniProtKB:Q8IZ41",
  "gene_name": "Ras and EF-hand domain-containing protein",
  "term_id": "GO:0016192"
}